{
  "gene_symbol": "CCNJL",
  "gene": "UniProtKB:Q8IV13",
  "term_id": "GO:0000082",
  "gene_name": "Cyclin-J-like protein",
  "term_label": "G1/S transition of mitotic cell cycle"
}